{
  "gene_symbol": "TWIST2",
  "gene": "UniProtKB:Q8WVJ9",
  "gene_name": "Twist-related protein 2",
  "term_id": "GO:0006357",
  "term_label": "regulation of transcription by RNA polymerase II"
}